{
  "gene_symbol": "TLR10",
  "term_label": "plasma membrane",
  "term_id": "GO:0005886",
  "gene": "UniProtKB:Q9BXR5",
  "gene_name": "Toll-like receptor 10"
}